{
  "term_label": "structural constituent of chromatin",
  "term_id": "GO:0030527",
  "gene": "UniProtKB:Q8N257",
  "gene_symbol": "H2BC26",
  "gene_name": "Histone H2B type 3-B"
}